{
  "gene": "UniProtKB:Q8TE73",
  "gene_symbol": "DNAH5",
  "term_id": "GO:0036157",
  "gene_name": "Dynein axonemal heavy chain 5",
  "term_label": "outer dynein arm"
}